U4atac/U6atac x U5 tri-snRNP complex [GO:0071009] (CC) References: PMID:16201866 Sources: GOC:krc, GOC:mah, GOC:pr, ISBN:0879695897 Definition: A spliceosomal snRNP complex that is formed by the association of the U4atac/U6atac and U5 snRNPs. Relationships: is a type of GO:0097526; has part U5 snRNP [GO:0005682]; has part U4atac/U6atac snRNP [GO:0071002] Also known as: U4atac/U6atac.U5 snRNP complex